{
  "term_id": "GO:0019722",
  "term_label": "calcium-mediated signaling",
  "gene": "UniProtKB:Q9GZZ8",
  "gene_symbol": "LACRT",
  "gene_name": "Extracellular glycoprotein lacritin"
}